positive regulation of shell calcification [GO:1905650] (biological process) Relationships: is a type of positive regulation of biomineral tissue development [GO:0070169]; is a type of regulation of shell calcification [GO:1905648]; positively regulates GO:0031215 References: PMID:14648763 Sources: GOC:TermGenie, GO_REF:0000058 Definition: Any process that activates or increases the frequency, rate or extent of shell calcification. Also known as: up regulation of shell calcification, up-regulation of shell calcification, upregulation of shell calcification, activation of shell calcification